{
  "term_label": "cytoplasm",
  "gene_name": "Developmental pluripotency-associated 5 protein",
  "gene": "UniProtKB:A6NC42",
  "gene_symbol": "DPPA5",
  "term_id": "GO:0005737"
}